{
  "gene_symbol": "CHRM1",
  "term_id": "GO:0007197",
  "term_label": "adenylate cyclase-inhibiting G protein-coupled acetylcholine receptor signaling pathway",
  "gene": "UniProtKB:P11229",
  "gene_name": "Muscarinic acetylcholine receptor M1"
}